{
  "term_label": "nucleus",
  "gene_symbol": "PSMA8",
  "gene": "UniProtKB:Q8TAA3",
  "term_id": "GO:0005634",
  "gene_name": "Proteasome subunit alpha-type 8"
}